negative regulation of mitochondrial ATP synthesis coupled electron transport [GO:1905447] (BP) Definition: Any process that stops, prevents or reduces the frequency, rate or extent of mitochondrial ATP synthesis coupled electron transport. Also known as: down regulation of mitochondrial ATP synthesis coupled electron transport, down-regulation of mitochondrial ATP synthesis coupled electron transport, downregulation of mitochondrial ATP synthesis coupled electron transport, inhibition of mitochondrial ATP synthesis coupled electron transport Relationships: is a type of negative regulation of oxidative phosphorylation [GO:0090324]; is a type of regulation of mitochondrial ATP synthesis coupled electron transport [GO:1905446]; negatively regulates mitochondrial ATP synthesis coupled electron transport [GO:0042775] Subtypes: negative regulation of mitochondrial electron transport, NADH to ubiquinone [GO:1902957] References: PMID:23707074 Sources: GOC:PARL, GOC:TermGenie, GOC:bc, GO_REF:0000058